{
  "gene_symbol": "RNASEH2A",
  "gene": "UniProtKB:O75792",
  "term_label": "RNA-DNA hybrid ribonuclease activity",
  "gene_name": "Ribonuclease H2 subunit A",
  "term_id": "GO:0004523"
}